{
  "term_id": "GO:0016324",
  "gene_symbol": "SLC15A2",
  "gene": "UniProtKB:Q16348",
  "gene_name": "Solute carrier family 15 member 2",
  "term_label": "apical plasma membrane"
}